regulation of organelle organization [GO:0033043] (biological process) Subtypes: regulation of COPII vesicle coating [GO:0003400], positive regulation of organelle organization [GO:0010638], negative regulation of organelle organization [GO:0010639], regulation of mitochondrion organization [GO:0010821], GO:0031338, regulation of chromosome organization [GO:0033044], regulation of vacuole organization [GO:0044088], regulation of cytoskeleton organization [GO:0051493], regulation of nuclear division [GO:0051783], regulation of synaptic vesicle budding from presynaptic endocytic zone membrane [GO:0098694], GO:1900063, regulation of autophagosome maturation [GO:1901096], regulation of organelle assembly [GO:1902115], GO:1903056, regulation of nucleus organization [GO:1903353], regulation of Golgi organization [GO:1903358], GO:1903371, regulation of secretory granule organization [GO:1904409], regulation of endosome organization [GO:1904978], regulation of phagosome maturation [GO:1905162], regulation of chloroplast fission [GO:1905192], GO:1905874 Sources: GOC:mah Relationships: is a type of regulation of cellular component organization [GO:0051128]; regulates organelle organization [GO:0006996] Also known as: regulation of organelle organisation, regulation of organelle organization and biogenesis Definition: Any process that modulates the frequency, rate or extent of a process involved in the formation, arrangement of constituent parts, or disassembly of an organelle.